SNARE complex [GO:0031201] (cellular component) Definition: A protein complex involved in membrane fusion; a stable ternary complex consisting of a four-helix bundle, usually formed from one R-SNARE and three Q-SNAREs with an ionic layer sandwiched between hydrophobic layers. One well-characterized example is the neuronal SNARE complex formed of synaptobrevin 2, syntaxin 1a, and SNAP-25. Subtypes: synaptobrevin 2-SNAP-25-syntaxin-1a-complexin I complex [GO:0070032], GO:0070033, GO:0070044, synaptobrevin 2-SNAP-25-syntaxin-2 complex [GO:0070045], synaptobrevin 2-SNAP-25-syntaxin-3 complex [GO:0070046], synaptobrevin 2-SNAP-25-syntaxin-4 complex [GO:0070047], endobrevin-SNAP-25-syntaxin-1a complex [GO:0070048], endobrevin-SNAP-25-syntaxin-2 complex [GO:0070049], cellubrevin-VAMP4-syntaxin-16 complex [GO:0070065], cellubrevin-VAMP4-endobrevin-syntaxin-6 complex [GO:0070066], GO:0070067, VAMP4-syntaxin-6-syntaxin-16-Vti1a complex [GO:0070068], synaptotagmin-synaptobrevin 2-SNAP-25-syntaxin-1a-syntaxin-1b-Rab3a-complexin II complex [GO:0070355], GO:0070356, synaptobrevin 2-SNAP-25-syntaxin-3-complexin complex [GO:0070554], endobrevin-synaptobrevin 2-alpha-SNAP-NSF-syntaxin-4 complex [GO:0070766], synaptotagmin-synaptobrevin 2-SNAP-25-syntaxin-1a-syntaxin-1b-Unc13 complex [GO:0070768], platelet SNARE complex [GO:0097654] Relationships: is a type of membrane protein complex [GO:0098796]; BFO_0000050 GO:0005737 References: PMID:10872468, PMID:19450911 Sources: GOC:bhm, GOC:pr